negative regulation of pyruvate decarboxylation to acetyl-CoA [GO:0160218] (biological process) Definition: Any process that stops, prevents or reduces the frequency, rate or extent of the chemical reactions and pathways resulting in the formation of acetyl-CoA from pyruvate. In most organisms, this pathway links glycolysis to the TCA cycle, by a series of three reactions carried out by a multisubunit complex called the 'pyruvate dehydrogenase complex', even though pyruvate dehydrogenase activity describes only one of those reactions. Relationships: is a type of GO:0009890; is a type of GO:0010510; is_a negative regulation of amide metabolic process [GO:0034249]; is a type of negative regulation of nucleobase-containing compound metabolic process [GO:0045934]; is a type of GO:0045936; is a type of GO:0062014; negatively regulates GO:0006086 References: PMID:26942675, PMID:36849569, PMID:37754565 Also known as: negative regulation of acetyl-CoA biosynthetic process from pyruvate